{
  "gene_name": "Cystatin-SA",
  "term_label": "Unknown biological process",
  "gene_symbol": "CST2",
  "gene": "UniProtKB:P09228",
  "term_id": "UNKNOWN:0002"
}